TIMP family protein binding [GO:0098769] (MF) References: PMID:22078297 Definition: Binding to a member of the Tissue inhibitors of metalloproteinases (TIMPs) family. TIMPs are endogenous protein regulators of the matrix metalloproteinase (MMPs) family. Relationships: is a type of protein binding [GO:0005515]